{
  "term_label": "nucleus",
  "term_id": "GO:0005634",
  "gene": "UniProtKB:Q9Y462",
  "gene_name": "Zinc finger protein 711",
  "gene_symbol": "ZNF711"
}